{
  "gene_name": "Eyes absent homolog 4",
  "term_label": "nucleus",
  "term_id": "GO:0005634",
  "gene": "UniProtKB:O95677",
  "gene_symbol": "EYA4"
}